{
  "gene_name": "Sodium_nucleoside cotransporter 2",
  "gene_symbol": "SLC28A2",
  "term_label": "plasma membrane",
  "gene": "UniProtKB:O43868",
  "term_id": "GO:0005886"
}